{
  "gene": "UniProtKB:Q8TA86",
  "gene_name": "Retinitis pigmentosa 9 protein",
  "term_id": "UNKNOWN:0002",
  "term_label": "Unknown biological process",
  "gene_symbol": "RP9"
}